type B pancreatic cell fate commitment [GO:0003327] (biological process) Relationships: is a type of epithelial cell fate commitment [GO:0072148]; BFO_0000050 GO:0003309 Sources: CL:0000169, GOC:dph Definition: The commitment of a cell to a type B pancreatic cell fate and its capacity to differentiate into a type B pancreatic cell. A type B pancreatic cell is a cell located towards center of the islets of Langerhans that secretes insulin. Also known as: pancreatic B cell fate commitment